{
  "gene": "UniProtKB:O75643",
  "term_id": "GO:0005681",
  "term_label": "spliceosomal complex",
  "gene_name": "U5 small nuclear ribonucleoprotein 200 kDa helicase",
  "gene_symbol": "SNRNP200"
}